glycolipid translocation [GO:0034203] (biological process) References: PMID:11807558 Sources: GOC:go_curators Relationships: is a type of lipid translocation [GO:0034204]; is a type of glycolipid transport [GO:0046836] Definition: The translocation, or flipping, of glycolipid molecules from one monolayer of a membrane bilayer to the opposite monolayer.